negative regulation of toll-like receptor 9 signaling pathway [GO:0034164] (biological process) Definition: Any process that stops, prevents, or reduces the frequency, rate, or extent of toll-like receptor 9 signaling pathway. References: PMID:16551253, PMID:17328678 Sources: GOC:add Also known as: negative regulation of TLR9 signaling pathway, negative regulation of toll-like receptor 9 signalling pathway Relationships: is a type of regulation of toll-like receptor 9 signaling pathway [GO:0034163]; is a type of negative regulation of cytoplasmic pattern recognition receptor signaling pathway [GO:0039532]; negatively regulates toll-like receptor 9 signaling pathway [GO:0034162]